{
  "term_label": "Unknown molecular function",
  "gene_symbol": "EDEM2",
  "gene": "UniProtKB:Q9BV94",
  "gene_name": "ER degradation-enhancing alpha-mannosidase-like protein 2",
  "term_id": "UNKNOWN:0001"
}